glucoside transport [GO:0042946] (biological process) Definition: The directed movement of glucosides into, out of or within a cell, or between cells, by means of some agent such as a transporter or pore. Glucosides are glycosides in which the sugar group is a glucose residue. Sources: GOC:jl, ISBN:0198506732 Relationships: is a type of GO:1901656 Subtypes: alpha-glucoside transport [GO:0000017], GO:0015759, GO:1902418